{
  "gene_name": "Adrenocorticotropic hormone receptor",
  "term_label": "adenylate cyclase-activating G protein-coupled receptor signaling pathway",
  "gene_symbol": "MC2R",
  "term_id": "GO:0007189",
  "gene": "UniProtKB:Q01718"
}